{
  "gene_name": "Erythroferrone",
  "gene": "UniProtKB:Q4G0M1",
  "term_id": "GO:0046326",
  "gene_symbol": "ERFE",
  "term_label": "positive regulation of D-glucose import"
}